L-lysine import into vacuole involved in cellular response to nitrogen starvation [GO:1901482] (biological process) Definition: A L-lysine import into the vacuole that is involved in cellular response to nitrogen starvation. Sources: GOC:TermGenie Relationships: is a type of L-lysine transmembrane import into vacuole [GO:0090517]; is part of cellular response to nitrogen starvation [GO:0006995]